{
  "gene": "UniProtKB:Q6ZMP0",
  "gene_symbol": "THSD4",
  "gene_name": "Thrombospondin type-1 domain-containing protein 4",
  "term_label": "Unknown cellular component",
  "term_id": "UNKNOWN:0003"
}